{
  "gene": "UniProtKB:P32019",
  "term_label": "Unknown biological process",
  "gene_name": "Type II inositol 1,4,5-trisphosphate 5-phosphatase",
  "term_id": "UNKNOWN:0002",
  "gene_symbol": "INPP5B"
}